C-4 methylsterol oxidase activity [GO:0000254] (molecular function) Also known as: 4-methylsterol oxidase activity, methylsterol hydroxylase activity, methylsterol monooxygenase activity References: PMID:9811880 Sources: RHEA:55220 Relationships: is a type of oxidoreductase activity, acting on paired donors, with incorporation or reduction of molecular oxygen, another compound as one donor, and incorporation of one atom of oxygen [GO:0016716] Definition: Catalysis of the reaction: 4,4-dimethyl-5alpha-cholest-7-en-3beta-ol + 6 Fe(II)-[cytochrome b5] + 5 H+ + 3 O2 = 4alpha-carboxy-4beta-methyl-5alpha-cholest-7-ene-3beta-ol + 6 Fe(III)-[cytochrome b5] + 4 H2O.